{
  "gene_symbol": "TCTN2",
  "gene_name": "Tectonic-2",
  "gene": "UniProtKB:Q96GX1",
  "term_label": "protein localization to ciliary transition zone",
  "term_id": "GO:1904491"
}